{
  "gene": "UniProtKB:Q9BQI6",
  "gene_name": "SMC5-SMC6 complex localization factor protein 1",
  "term_label": "site of double-strand break",
  "term_id": "GO:0035861",
  "gene_symbol": "SLF1"
}